{
  "gene_name": "Protein FAM177A1",
  "gene": "UniProtKB:Q8N128",
  "gene_symbol": "FAM177A1",
  "term_id": "UNKNOWN:0003",
  "term_label": "Unknown cellular component"
}